{
  "term_label": "D-glucose import across plasma membrane",
  "term_id": "GO:0098708",
  "gene_symbol": "SLC5A4",
  "gene": "UniProtKB:Q9NY91",
  "gene_name": "Probable glucose sensor protein SLC5A4"
}